esculetin biosynthetic process [GO:0033493] (biological process) Definition: The chemical reactions and pathways resulting in the formation of esculetin, 6,7-dihydroxycoumarin. Also known as: esculetin anabolism, esculetin biosynthesis, esculetin formation, esculetin synthesis Relationships: is a type of coumarin biosynthetic process [GO:0009805] Sources: GOC:mah